{
  "gene": "UniProtKB:Q8TC94",
  "gene_symbol": "ACTL9",
  "term_label": "actin cytoskeleton",
  "gene_name": "Actin-like protein 9",
  "term_id": "GO:0015629"
}